positive regulation of lyase activity [GO:0051349] (biological process) Definition: Any process that activates or increases the frequency, rate or extent of lyase activity, the catalysis of the cleavage of C-C, C-O, C-N and other bonds by other means than by hydrolysis or oxidation, or conversely adding a group to a double bond. Subtypes: positive regulation of guanylate cyclase activity [GO:0031284], positive regulation of adenylate cyclase activity [GO:0045762] Also known as: lyase activator, up regulation of lyase activity, up-regulation of lyase activity, upregulation of lyase activity, activation of lyase activity, stimulation of lyase activity Relationships: is a type of positive regulation of catalytic activity [GO:0043085]; positively regulates GO:0016829 Sources: GOC:ai